protein-lipid complex organization [GO:0071825] (biological process) Also known as: protein-lipid complex subunit organisation, protein-lipid complex subunit organization Definition: Any process in which macromolecules aggregate, disaggregate, or are modified, resulting in the formation, disassembly, or alteration of a protein-lipid complex. Relationships: is a type of GO:0043933 Sources: GOC:mah Subtypes: protein-lipid complex disassembly [GO:0032987], GO:0034368, protein-lipid complex assembly [GO:0065005], plasma lipoprotein particle organization [GO:0071827]